{
  "gene_name": "Putative olfactory receptor 2B3",
  "term_label": "plasma membrane",
  "term_id": "GO:0005886",
  "gene_symbol": "OR2B3",
  "gene": "UniProtKB:O76000"
}